{
  "gene_name": "BMP-2-inducible protein kinase",
  "term_label": "positive regulation of Notch signaling pathway",
  "gene": "UniProtKB:Q9NSY1",
  "term_id": "GO:0045747",
  "gene_symbol": "BMP2K"
}